{
  "gene_name": "Probable tubulin polyglutamylase TTLL2",
  "gene_symbol": "TTLL2",
  "gene": "UniProtKB:Q9BWV7",
  "term_label": "microtubule cytoskeleton organization",
  "term_id": "GO:0000226"
}